{
  "gene_symbol": "FBN3",
  "term_label": "hormone activity",
  "gene_name": "Fibrillin-3",
  "term_id": "GO:0005179",
  "gene": "UniProtKB:Q75N90"
}